{
  "gene": "UniProtKB:Q9BQY9",
  "term_label": "Unknown cellular component",
  "gene_symbol": "DBNDD2",
  "term_id": "UNKNOWN:0003",
  "gene_name": "Dysbindin domain-containing protein 2"
}